{
  "gene_name": "Receptor-transporting protein 3",
  "gene_symbol": "RTP3",
  "term_id": "GO:0031849",
  "gene": "UniProtKB:Q9BQQ7",
  "term_label": "olfactory receptor binding"
}